xylosyl alpha-1,3-xylosyltransferase activity [GO:0140560] (molecular function) References: PMID:22117070, PMID:8982869 Sources: RHEA:22820 Relationships: is a type of UDP-xylosyltransferase activity [GO:0035252] Definition: Catalyzes the reaction: UDP-alpha-D-xylose + [protein with EGF-like domain]-3-O-(alpha-D-xylosyl-(1->3)-beta-D-glucosyl)-L-serine = UDP + [protein with EGF-like domain]-3-O-(alpha-D-xylosyl-(1->3)-alpha-D-xylosyl-(1->3)-beta-D-glucosyl)-L-serine. The enzyme, found in animals and insects, is involved in the biosynthesis of the alpha-D-xylosyl-(1->3)-alpha-D-xylosyl-(1->3)- beta-D-glucosyl trisaccharide on epidermal growth factor-like (EGF- like) domains.